cell differentiation involved in salivary gland development [GO:0060689] (biological process) Sources: GOC:dph Subtypes: GO:0060690, mesenchymal cell differentiation involved in salivary gland development [GO:0060692], neuron differentiation involved in salivary gland development [GO:0060705] Relationships: is_a cell differentiation [GO:0030154]; is part of salivary gland development [GO:0007431] Definition: The process in which a relatively unspecialized cell acquires specialized structural and/or functional features that characterize the cells of the salivary gland.